{
  "gene": "UniProtKB:O60318",
  "gene_symbol": "MCM3AP",
  "term_label": "Unknown molecular function",
  "gene_name": "Germinal-center associated nuclear protein",
  "term_id": "UNKNOWN:0001"
}